UDP-N-acetylgalactosamine diphosphorylase activity [GO:0052630] (molecular function) Definition: Catalysis of the reaction: UTP + N-acetyl-alpha-D-galactosamine 1-phosphate = diphosphate + UDP-N-acetyl-D-galactosamine. Relationships: is a type of uridylyltransferase activity [GO:0070569] Also known as: N-acetylgalactosamine 1-phosphate uridylyltransferase, N-acetylgalactosamine-1-phosphate uridyltransferase activity, UDP-GalNAc pyrophosphorylase activity, UDP-N-acetylgalactosamine pyrophosphorylase activity, UDP-acetylgalactosamine pyrophosphorylase activity, UTP:2-acetamido-2-deoxy-alpha-D-galactose-1-phosphate uridylyltransferase activity, UTP:N-acetyl-alpha-D-galactosamine-1-phosphate uridylyltransferase activity, uridine diphosphate-N-acetylgalactosamine pyrophosphorylase activity, uridine diphosphoacetylgalactosamine phosphorylase activity, uridine diphosphoacetylgalactosamine pyrophosphorylase activity Sources: EC:2.7.7.83, RHEA:34363